{
  "gene_symbol": "CDK18",
  "gene": "UniProtKB:Q07002",
  "gene_name": "Cyclin-dependent kinase 18",
  "term_label": "cyclin-dependent protein kinase holoenzyme complex",
  "term_id": "GO:0000307"
}